protein-containing complex binding [GO:0044877] (molecular function) Subtypes: TFIIA-class transcription factor complex binding [GO:0001092], GO:0001094, TFIIE-class transcription factor complex binding [GO:0001095], TFIIF-class transcription factor complex binding [GO:0001096], GO:0001097, complement component C1q complex binding [GO:0001849], type I interferon receptor binding [GO:0005132], integrin binding [GO:0005178], collagen binding [GO:0005518], anaphase-promoting complex binding [GO:0010997], immunoglobulin binding [GO:0019865], MHC protein complex binding [GO:0023023], GO:0030507, GO:0031491, G-protein beta/gamma-subunit complex binding [GO:0031683], GO:0032404, heterotrimeric G-protein binding [GO:0032795], inhibin complex binding [GO:0034710], Fc-gamma receptor I complex binding [GO:0034988], AP-2 adaptor complex binding [GO:0035612], AP-1 adaptor complex binding [GO:0035650], AP-3 adaptor complex binding [GO:0035651], GO:0036033, BLOC-2 complex binding [GO:0036461], GO:0042608, ribonucleoprotein complex binding [GO:0043021], GO:0048185, GO:0051015, transcription factor TFIIH holo complex binding [GO:0062058], GO:0062059, GO:0062060, GO:0062061, GO:0062062, BBSome binding [GO:0062063], PSII associated light-harvesting complex II binding [GO:0062066], GO:0062067, chloroplast photosystem II binding [GO:0062068], GARP complex binding [GO:0062069], GO:0062070, TSC1-TSC2 complex binding [GO:0062078], fibrinogen binding [GO:0070051], GO:0070628, GO:0070840, protein-lipid complex binding [GO:0071814], Arp2/3 complex binding [GO:0071933], GO:0106080, IkappaB kinase complex binding [GO:0106137], Sec61 translocon complex binding [GO:0106138], P-TEFb complex binding [GO:0106140], GO:0120160, intraciliary transport particle B binding [GO:0120170], NuRD complex binding [GO:0120325], Golgi transport complex binding [GO:0140164], PRC1 complex binding [GO:0140259], mitochondrial proton-transporting ATP synthase complex binding [GO:0140260], mRNA cap binding complex binding [GO:0140262], GO:0140496, BAT3 complex binding [GO:1904288], beta-catenin destruction complex binding [GO:1904713], GO:1904841, proteasome core complex binding [GO:1904854], proteasome regulatory particle binding [GO:1904855], MCM complex binding [GO:1904931], GO:1905334, retromer complex binding [GO:1905394], SCF ubiquitin ligase complex binding [GO:1905761], GO:1905762, MTREC complex binding [GO:1905763], exon-exon junction complex binding [GO:1990448], GO:1990593 Definition: Binding to a macromolecular complex. Sources: GOC:jl Also known as: protein complex binding, macromolecular complex binding Relationships: is a type of binding [GO:0005488]